{
  "gene_symbol": "LIPC",
  "term_label": "cholesterol homeostasis",
  "term_id": "GO:0042632",
  "gene": "UniProtKB:P11150",
  "gene_name": "Hepatic triacylglycerol lipase"
}